{
  "gene_symbol": "ZNF718",
  "term_id": "GO:0006355",
  "gene": "UniProtKB:Q3SXZ3",
  "gene_name": "Zinc finger protein 718",
  "term_label": "regulation of DNA-templated transcription"
}